{
  "gene_name": "POTE ankyrin domain family member A",
  "gene_symbol": "POTEA",
  "term_id": "UNKNOWN:0003",
  "gene": "UniProtKB:Q6S8J7",
  "term_label": "Unknown cellular component"
}